{
  "term_id": "UNKNOWN:0003",
  "gene_name": "Adhesion G-protein coupled receptor F3",
  "gene_symbol": "ADGRF3",
  "gene": "UniProtKB:Q8IZF5",
  "term_label": "Unknown cellular component"
}